{
  "term_id": "GO:0035267",
  "term_label": "NuA4 histone acetyltransferase complex",
  "gene_symbol": "ING3",
  "gene": "UniProtKB:Q9NXR8",
  "gene_name": "Inhibitor of growth protein 3"
}